immunoglobulin production involved in immunoglobulin-mediated immune response [GO:0002381] (biological process) Definition: The appearance of immunoglobulin due to biosynthesis or secretion following a cellular stimulus during an immune response, resulting in an increase in its intracellular or extracellular levels. Subtypes: immunoglobulin production in mucosal tissue [GO:0002426] Also known as: immunoglobulin production involved in immunoglobulin mediated immune response, immunoglobulin biosynthetic process involved in immune response, immunoglobulin secretion involved in immune response, antibody production during immune response, antibody secretion during immune response, immunoglobulin production during immune response, immunoglobulin production involved in immune response References: PMID:9185563 Sources: GOC:add, ISBN:0781735149 Relationships: is a type of GO:0002377; is part of immunoglobulin mediated immune response [GO:0016064] Note: Note that this term is in the subset of terms that should not be used for direct gene product annotation. Instead, select one of the 'regulation' children terms.